4-hydroxyphenylacetate biosynthetic process [GO:1901024] (biological process) Definition: The chemical reactions and pathways resulting in the formation of 4-hydroxyphenylacetate. Sources: GOC:TermGenie, GOC:yaf Also known as: 4-hydroxyphenylacetate anabolism, 4-hydroxyphenylacetate biosynthesis, 4-hydroxyphenylacetate formation, 4-hydroxyphenylacetate synthesis Relationships: is a type of GO:0046189; is_a monocarboxylic acid biosynthetic process [GO:0072330]; is a type of 4-hydroxyphenylacetate metabolic process [GO:1901022]